methane-oxidizing organelle [GO:0044227] (cellular component) Definition: A cytoplasmic, membrane-bounded compartment found within Methanotrophic bacteria that contains enzymes and electron transfer proteins for methane catabolism. This structure is analogous to the thylakoid of Cyanobacteria and the anammoxosome of anaerobic ammonium oxidation organisms. Sources: GOC:dh Also known as: methane-oxidizing compartment, methanotroph intracytoplasmic membrane-bound compartment Relationships: is a type of intracellular membrane-bounded organelle [GO:0043231]; BFO_0000050 cytoplasm [GO:0005737]